{
  "gene_symbol": "LITAFD",
  "gene": "UniProtKB:A0A1B0GVX0",
  "gene_name": "LITAF domain-containing protein",
  "term_id": "GO:0098560",
  "term_label": "cytoplasmic side of late endosome membrane"
}